{
  "term_label": "Unknown biological process",
  "gene_name": "Interphotoreceptor matrix proteoglycan 1",
  "gene_symbol": "IMPG1",
  "term_id": "UNKNOWN:0002",
  "gene": "UniProtKB:Q17R60"
}